maleate isomerase activity [GO:0050076] (molecular function) Relationships: is a type of cis-trans isomerase activity [GO:0016859] Definition: Catalysis of the reaction: maleate = fumarate. Sources: EC:5.2.1.1, RHEA:13169 Also known as: maleate cis-trans-isomerase activity